pyridoxal phosphate metabolic process [GO:0042822] (biological process) Sources: GOC:jl Relationships: is a type of aldehyde metabolic process [GO:0006081]; is a type of GO:0006796; is a type of organophosphate metabolic process [GO:0019637]; is a type of GO:0042816 Also known as: active vitamin B6 metabolic process, active vitamin B6 metabolism, pyridoxal phosphate metabolism Definition: The chemical reactions and pathways involving pyridoxal phosphate, pyridoxal phosphorylated at the hydroxymethyl group of C-5, the active form of vitamin B6. Subtypes: pyridoxal phosphate catabolic process [GO:0032361], pyridoxal phosphate biosynthetic process [GO:0042823]